{
  "term_label": "Unknown cellular component",
  "gene_symbol": "FKSG35",
  "gene_name": "FKSG35",
  "gene": "UniProtKB:Q9BZC5",
  "term_id": "UNKNOWN:0003"
}